{
  "gene_name": "Ubiquitin-like protein ATG12",
  "gene_symbol": "ATG12",
  "term_label": "autophagosome membrane",
  "gene": "UniProtKB:O94817",
  "term_id": "GO:0000421"
}